{
  "gene_name": "Propionyl-CoA carboxylase beta chain, mitochondrial",
  "gene": "UniProtKB:P05166",
  "term_label": "mitochondrion",
  "term_id": "GO:0005739",
  "gene_symbol": "PCCB"
}